DNA transmembrane transporter activity [GO:0051035] (molecular function) Definition: Enables the transfer of DNA, deoxyribonucleic acid, from one side of a membrane to the other. Sources: GOC:ai Relationships: is a type of nucleic acid transmembrane transporter activity [GO:0051032]; is part of DNA transport [GO:0051027]